{
  "term_id": "GO:0043235",
  "term_label": "receptor complex",
  "gene_name": "Tyrosine-protein kinase transmembrane receptor ROR2",
  "gene_symbol": "ROR2",
  "gene": "UniProtKB:Q01974"
}